{
  "term_label": "plasma membrane",
  "gene": "UniProtKB:Q99653",
  "gene_symbol": "CHP1",
  "gene_name": "Calcineurin B homologous protein 1",
  "term_id": "GO:0005886"
}